lysine:proton symporter activity [GO:0015493] (molecular function) Also known as: lysine:hydrogen symporter activity Relationships: is a type of amino acid:proton symporter activity [GO:0005280]; is a type of carboxylic acid transmembrane transporter activity [GO:0046943] Sources: TC:2.A.3.1.2 Definition: Enables the transfer of a solute or solutes from one side of a membrane to the other according to the reaction: lysine(out) + H+(out) = lysine(in) + H+(in).